{
  "term_id": "GO:0071916",
  "gene_symbol": "SLC15A1",
  "gene_name": "Solute carrier family 15 member 1",
  "term_label": "dipeptide transmembrane transporter activity",
  "gene": "UniProtKB:P46059"
}